T cell receptor signaling pathway [GO:0050852] (biological process) Also known as: T lymphocyte receptor signaling pathway, T lymphocyte receptor signalling pathway, T-cell receptor signaling pathway, T-cell receptor signalling pathway, T-lymphocyte receptor signaling pathway, T-lymphocyte receptor signalling pathway, TCR signaling pathway Regulation: regulated by regulation of T cell receptor signaling pathway [GO:0050856]; negatively regulated by GO:0050860; positively regulated by positive regulation of T cell receptor signaling pathway [GO:0050862] Sources: GOC:add Relationships: is a type of antigen receptor-mediated signaling pathway [GO:0050851] Definition: The series of molecular signals initiated by the cross-linking of an antigen receptor on a T cell.